{
  "gene": "UniProtKB:Q9H3S4",
  "gene_name": "Thiamin pyrophosphokinase 1",
  "term_id": "GO:0009229",
  "gene_symbol": "TPK1",
  "term_label": "thiamine diphosphate biosynthetic process"
}